{
  "gene": "UniProtKB:Q96MM3",
  "gene_symbol": "ZFP42",
  "gene_name": "Zinc finger protein 42 homolog",
  "term_label": "regulation of transcription by RNA polymerase II",
  "term_id": "GO:0006357"
}